{
  "gene_name": "TATA-binding protein-associated factor 2N",
  "term_label": "transcription coregulator activity",
  "term_id": "GO:0003712",
  "gene_symbol": "TAF15",
  "gene": "UniProtKB:Q92804"
}